{
  "term_label": "cytosol",
  "term_id": "GO:0005829",
  "gene": "UniProtKB:P09455",
  "gene_name": "Retinol-binding protein 1",
  "gene_symbol": "RBP1"
}